{
  "term_label": "autophagosome-lysosome fusion",
  "term_id": "GO:0061909",
  "gene_name": "Protein associated with UVRAG as autophagy enhancer",
  "gene_symbol": "RUBCNL",
  "gene": "UniProtKB:Q9H714"
}